collagen type XX trimer [GO:1990319] (cellular component) References: PMID:17876790 Definition: A collagen homotrimer of alpha1(XX) chains. Relationships: is a type of GO:0005593